{
  "gene_name": "CD320 antigen",
  "term_id": "GO:0005886",
  "term_label": "plasma membrane",
  "gene_symbol": "CD320",
  "gene": "UniProtKB:Q9NPF0"
}